quercetin 3-O-methyltransferase activity [GO:0030755] (molecular function) Also known as: S-adenosyl-L-methionine:3,5,7,3',4'-pentahydroxyflavone 3-O-methyltransferase activity, flavonoid 3-methyltransferase activity, flavonol 3-O-methyltransferase activity Sources: EC:2.1.1.76 Relationships: is a type of S-adenosylmethionine-dependent methyltransferase activity [GO:0008757] Definition: Catalysis of the reaction: S-adenosyl-L-methionine + 3,5,7,3',4'-pentahydroxyflavone = S-adenosyl-L-homocysteine + 3-methoxy-5,7,3',4'-tetrahydroxy-flavone.